{
  "term_id": "GO:0004305",
  "gene_name": "Choline_ethanolamine kinase",
  "gene_symbol": "CHKB",
  "term_label": "ethanolamine kinase activity",
  "gene": "UniProtKB:Q9Y259"
}